peptidyl-amino acid modification [GO:0018193] (biological process) Relationships: is a type of protein modification process [GO:0036211] Subtypes: peptidyl-L-amino acid racemization [GO:0018085], peptidyl-alanine modification [GO:0018194], peptidyl-arginine modification [GO:0018195], peptidyl-aspartic acid modification [GO:0018197], peptidyl-cysteine modification [GO:0018198], peptidyl-glutamine modification [GO:0018199], GO:0018200, GO:0018201, peptidyl-histidine modification [GO:0018202], peptidyl-isoleucine modification [GO:0018203], peptidyl-leucine modification [GO:0018204], peptidyl-lysine modification [GO:0018205], peptidyl-methionine modification [GO:0018206], peptidyl-phenylalanine modification [GO:0018207], peptidyl-proline modification [GO:0018208], peptidyl-serine modification [GO:0018209], peptidyl-threonine modification [GO:0018210], peptidyl-tryptophan modification [GO:0018211], GO:0018212, peptidyl-valine modification [GO:0018213], GO:0050844 Definition: The alteration of an amino acid residue in a peptide. Sources: GOC:mah